{
  "gene": "UniProtKB:Q9NP86",
  "gene_symbol": "CABP5",
  "term_id": "GO:0005246",
  "term_label": "calcium channel regulator activity",
  "gene_name": "Calcium-binding protein 5"
}